{
  "term_label": "plasma membrane",
  "gene_symbol": "RAB5B",
  "gene": "UniProtKB:P61020",
  "gene_name": "Ras-related protein Rab-5B",
  "term_id": "GO:0005886"
}